{
  "term_label": "protein localization to endoplasmic reticulum exit site",
  "gene_name": "B-cell receptor-associated protein 29",
  "gene_symbol": "BCAP29",
  "term_id": "GO:0070973",
  "gene": "UniProtKB:Q9UHQ4"
}